embryonic anterior midgut (ectodermal) morphogenesis [GO:0048615] (biological process) Definition: The process in which the anatomical structures of the anterior midgut (ectodermal) are generated and organized, during the embryonic phase. Relationships: is a type of morphogenesis of embryonic epithelium [GO:0016331]; is part of GO:0007441; is part of embryonic ectodermal digestive tract morphogenesis [GO:0048613] Sources: GOC:jid, GOC:rc